ribonucleoside biosynthetic process [GO:0042455] (biological process) Also known as: ribonucleoside anabolism, ribonucleoside biosynthesis, ribonucleoside formation, ribonucleoside synthesis Subtypes: purine ribonucleoside biosynthetic process [GO:0046129], pyrimidine ribonucleoside biosynthetic process [GO:0046132] Definition: The chemical reactions and pathways resulting in the formation of any ribonucleoside, a nucleoside in which purine or pyrimidine base is linked to a ribose (beta-D-ribofuranose) molecule. Relationships: is a type of ribonucleoside metabolic process [GO:0009119]; is a type of GO:0009163 Sources: GOC:jl